{
  "term_label": "RNA polymerase II cis-regulatory region sequence-specific DNA binding",
  "gene_name": "Zinc finger protein 304",
  "gene_symbol": "ZNF304",
  "term_id": "GO:0000978",
  "gene": "UniProtKB:Q9HCX3"
}